regulation of follicle-stimulating hormone secretion [GO:0046880] (BP) Definition: Any process that modulates the frequency, rate or extent of the regulated release of follicle-stimulating hormone. Also known as: regulation of FSH secretion, regulation of follicle stimulating hormone secretion Sources: GOC:ai Subtypes: positive regulation of follicle-stimulating hormone secretion [GO:0046881], negative regulation of follicle-stimulating hormone secretion [GO:0046882] Relationships: is a type of regulation of gonadotropin secretion [GO:0032276]; regulates follicle-stimulating hormone secretion [GO:0046884]